{
  "gene": "UniProtKB:Q9C0J9",
  "term_id": "GO:0000978",
  "term_label": "RNA polymerase II cis-regulatory region sequence-specific DNA binding",
  "gene_name": "Class E basic helix-loop-helix protein 41",
  "gene_symbol": "BHLHE41"
}